{
  "gene": "UniProtKB:Q5T5S1",
  "term_id": "UNKNOWN:0001",
  "term_label": "Unknown molecular function",
  "gene_symbol": "CCDC183",
  "gene_name": "Coiled-coil domain-containing protein 183"
}